sterol ester esterase activity [GO:0004771] (molecular function) Also known as: sterol esterase activity, cholesterol ester synthase activity, cholesterol esterase activity, acylcholesterol lipase activity, cholesterase activity, cholesterol ester hydrolase activity, cholesteryl ester hydrolase activity, cholesteryl ester synthase activity, cholesteryl esterase activity, sterol ester hydrolase activity, steryl-ester acylhydrolase activity, triterpenol esterase activity Sources: RHEA:10100 Definition: Catalysis of the reaction: a sterol ester + H2O = a fatty acid + a sterol + H+. Relationships: is a type of lipase activity [GO:0016298]; is a type of carboxylic ester hydrolase activity [GO:0052689]